symmetric cell division [GO:0098725] (biological process) Subtypes: symmetric stem cell division [GO:0098724] Definition: Cell division in which both daughter cells are of the same type. Relationships: is a type of cell division [GO:0051301] Sources: GOC:dos